reductive tricarboxylic acid cycle [GO:0019643] (biological process) Definition: A pathway leading to the fixation of two molecules of CO2 and the production of one molecule of acetyl-CoA; essentially the oxidative TCA cycle running in reverse. Acetyl-CoA is reductively carboxylated to pyruvate, from which all other central metabolites can be formed. Most of the enzymes of reductive and oxidative TCA cycle are shared, with the exception of three key enzymes that allow the cycle to run in reverse: ATP citrate lyase, 2-oxoglutarate:ferredoxin oxidoreductase, and fumarate reductase. 2-oxoglutarate:ferredoxin oxidoreductase catalyzes the carboxylation of succinyl-CoA to 2-oxoglutarate, ATP citrate lyase the ATP-dependent cleavage of citrate to acetyl-CoA and oxaloacetate, and fumarate reductase the reduction of fumarate forming succinate. References: PMID:15838028 Sources: GOC:jl Also known as: reductive Kreb's cycle, reductive TCA cycle, reductive carboxylate cycle, reductive carboxylic acid cycle, reductive citric acid pathway Relationships: is a type of carbon fixation [GO:0015977]